{
  "term_label": "3'-UTR-mediated mRNA stabilization",
  "gene_symbol": "ELAVL4",
  "gene": "UniProtKB:P26378",
  "gene_name": "ELAV-like protein 4",
  "term_id": "GO:0070935"
}